{
  "term_id": "GO:1901673",
  "gene": "UniProtKB:P12270",
  "gene_name": "Nucleoprotein TPR",
  "term_label": "regulation of mitotic spindle assembly",
  "gene_symbol": "TPR"
}